{
  "term_id": "GO:0000398",
  "gene": "UniProtKB:P0DJD4",
  "term_label": "mRNA splicing, via spliceosome",
  "gene_name": "RNA-binding motif protein, Y chromosome, family 1 member C",
  "gene_symbol": "RBMY1C"
}